{
  "term_label": "cytosol",
  "gene_symbol": "RBMS2",
  "gene": "UniProtKB:Q15434",
  "gene_name": "RNA-binding motif, single-stranded-interacting protein 2",
  "term_id": "GO:0005829"
}